{
  "term_label": "extracellular matrix",
  "gene_symbol": "COL21A1",
  "gene": "UniProtKB:Q96P44",
  "gene_name": "Collagen alpha-1(XXI) chain",
  "term_id": "GO:0031012"
}